{
  "gene": "UniProtKB:Q13795",
  "gene_name": "ADP-ribosylation factor-related protein 1",
  "term_label": "GTP binding",
  "gene_symbol": "ARFRP1",
  "term_id": "GO:0005525"
}